{
  "gene_symbol": "CRIPTO3",
  "term_id": "GO:0007368",
  "gene_name": "Putative teratocarcinoma-derived growth factor 3",
  "term_label": "determination of left/right symmetry",
  "gene": "UniProtKB:P51864"
}